D-alanine metabolic process [GO:0046436] (biological process) Subtypes: GO:0030632, D-alanine catabolic process [GO:0055130] Also known as: D-alanine metabolism Definition: The chemical reactions and pathways involving D-alanine, the D-enantiomer of the amino acid alanine, i.e. (2R)-2-aminopropanoic acid. Relationships: is a type of GO:0006522; is a type of D-amino acid metabolic process [GO:0046416] Sources: GOC:ai, GOC:jsg